leukocyte activation [GO:0045321] (biological process) Relationships: is a type of cell activation [GO:0001775]; is a type of immune system process [GO:0002376] Sources: GOC:add Subtypes: leukocyte activation involved in inflammatory response [GO:0002269], plasmacytoid dendritic cell activation [GO:0002270], myeloid leukocyte activation [GO:0002274], leukocyte activation involved in immune response [GO:0002366], lymphocyte activation [GO:0046649], GO:0050902 Definition: A change in morphology and behavior of a leukocyte resulting from exposure to a specific antigen, mitogen, cytokine, cellular ligand, or soluble factor. Also known as: immune cell activation, leucocyte activation Regulation: regulated by regulation of leukocyte activation [GO:0002694]; negatively regulated by negative regulation of leukocyte activation [GO:0002695]; RO_0002213 by positive regulation of leukocyte activation [GO:0002696]